{
  "gene_symbol": "ACP4",
  "term_label": "lysosome",
  "gene_name": "Testicular acid phosphatase",
  "term_id": "GO:0005764",
  "gene": "UniProtKB:Q9BZG2"
}